{
  "term_id": "UNKNOWN:0001",
  "gene_name": "BLOC-1-related complex subunit 6",
  "term_label": "Unknown molecular function",
  "gene_symbol": "BORCS6",
  "gene": "UniProtKB:Q96GS4"
}